hypoxanthine catabolic process [GO:0009114] (biological process) References: PMID:3196295 Also known as: hypoxanthine breakdown, hypoxanthine catabolism, hypoxanthine degradation, hypoxanthine oxidation Relationships: is a type of GO:0006145; is a type of GO:0046100 Definition: The chemical reactions and pathways resulting in the breakdown of hypoxanthine, 6-hydroxy purine, an intermediate in the degradation of adenylate. Its ribonucleoside is known as inosine and its ribonucleotide as inosinate.